regulation of systemic arterial blood pressure by neurotransmitter [GO:0003070] (biological process) Definition: The regulation of blood pressure mediated by a neurotransmitter. A neurotransmitter is any of a group of substances that are released on excitation from the axon terminal of a presynaptic neuron of the central or peripheral nervous system and travel across the synaptic cleft to either excite or inhibit the target cell. Relationships: is a type of nervous system process involved in regulation of systemic arterial blood pressure [GO:0001976]; is a type of regulation of systemic arterial blood pressure mediated by a chemical signal [GO:0003044] Sources: GOC:mtg_cardio Subtypes: regulation of systemic arterial blood pressure by acetylcholine [GO:0003068]